{
  "gene_symbol": "GMPPB",
  "term_id": "GO:0009298",
  "gene": "UniProtKB:Q9Y5P6",
  "gene_name": "Mannose-1-phosphate guanyltransferase beta",
  "term_label": "GDP-mannose biosynthetic process"
}